1,3-beta-D-glucan phosphorylase activity [GO:0047514] (molecular function) Definition: Catalysis of the reaction: [(1->3)-beta-D-glucosyl](n) + phosphate = [(1->3)-beta-D-glucosyl](n-1) + alpha-D-glucose 1-phosphate; substrates include laminarin. Sources: EC:2.4.1.97, MetaCyc:13-BETA-GLUCAN-PHOSPHORYLASE-RXN Relationships: is a type of hexosyltransferase activity [GO:0016758] Also known as: 1,3-beta-glucan phosphorylase activity, 1,3-beta-D-glucan:orthophosphate glucosyltransferase activity, 1,3-beta-D-glucan:phosphate alpha-D-glucosyltransferase activity, laminarin phosphorylase activity, laminarin phosphoryltransferase activity